{
  "gene_symbol": "TNFSF13B",
  "gene_name": "Tumor necrosis factor ligand superfamily member 13B",
  "term_id": "GO:0005125",
  "gene": "UniProtKB:Q9Y275",
  "term_label": "cytokine activity"
}